{
  "gene": "UniProtKB:Q8WWL2",
  "term_label": "establishment of meiotic spindle localization",
  "gene_name": "Protein spire homolog 2",
  "gene_symbol": "SPIRE2",
  "term_id": "GO:0051295"
}